plasma membrane bounded cell projection assembly [GO:0120031] (biological process) Definition: Formation of a prolongation or process extending and that is bounded by plasma membrane, e.g. a cilium, lamellipodium, or axon. Subtypes: substrate-dependent cell migration, cell extension [GO:0006930], extension of leading cell process to pial surface [GO:0021803], lamellipodium assembly [GO:0030032], microvillus assembly [GO:0030033], GO:0030035, pseudopodium assembly [GO:0031269], GO:0031382, bleb assembly [GO:0032060], uropod assembly [GO:0034460], cytoneme assembly [GO:0035231], GO:0046847, GO:0060271, dendritic cell dendrite assembly [GO:0097026], ruffle assembly [GO:0097178] Relationships: is a type of GO:0030031; is a type of plasma membrane bounded cell projection organization [GO:0120036] Sources: GOC:krc Regulation: regulated by GO:0120032; negatively regulated by negative regulation of plasma membrane bounded cell projection assembly [GO:0120033]; positively regulated by GO:0120034 Also known as: eupodium